{
  "gene_name": "Ubiquitin carboxyl-terminal hydrolase 15",
  "gene_symbol": "USP15",
  "term_label": "nucleus",
  "gene": "UniProtKB:Q9Y4E8",
  "term_id": "GO:0005634"
}